{
  "gene_name": "Ras-related protein Rab-43",
  "term_label": "endomembrane system",
  "gene_symbol": "RAB43",
  "term_id": "GO:0012505",
  "gene": "UniProtKB:Q86YS6"
}